W-molybdopterin cofactor catabolic process [GO:0032327] (biological process) Sources: GOC:mah Also known as: Moco catabolic process, Moco catabolism, W-molybdopterin cofactor breakdown, W-molybdopterin cofactor catabolism, W-molybdopterin cofactor degradation Definition: The chemical reactions and pathways resulting in the breakdown of the W-molybdopterin cofactor, essential for the catalytic activity of some enzymes. The cofactor consists of a mononuclear tungsten ion (W) coordinated by one or two molybdopterin ligands. Relationships: is_a molybdopterin cofactor catabolic process [GO:0032325]